{
  "gene_name": "Hypoxanthine-guanine phosphoribosyltransferase",
  "gene": "UniProtKB:P00492",
  "gene_symbol": "HPRT1",
  "term_label": "magnesium ion binding",
  "term_id": "GO:0000287"
}